{
  "term_id": "GO:0005886",
  "gene_symbol": "DUSP15",
  "gene": "UniProtKB:Q9H1R2",
  "term_label": "plasma membrane",
  "gene_name": "Dual specificity protein phosphatase 15"
}